{
  "term_id": "GO:0000981",
  "term_label": "DNA-binding transcription factor activity, RNA polymerase II-specific",
  "gene": "UniProtKB:P13682",
  "gene_symbol": "ZNF35",
  "gene_name": "Zinc finger protein 35"
}